{
  "gene": "UniProtKB:Q9UKP6",
  "term_label": "urotensin II receptor activity",
  "gene_symbol": "UTS2R",
  "term_id": "GO:0001604",
  "gene_name": "Urotensin-2 receptor"
}